{
  "gene_name": "eIF-2-alpha kinase GCN2",
  "gene": "UniProtKB:Q9P2K8",
  "term_label": "cellular response to amino acid starvation",
  "term_id": "GO:0034198",
  "gene_symbol": "EIF2AK4"
}